phosphatidylcholine-sterol O-acyltransferase activator activity [GO:0060228] (molecular function) Definition: Binds to and increases the activity of phosphatidylcholine-sterol O-acyltransferase. References: PMID:4335615 Sources: GOC:BHF, GOC:dph, GOC:tb Also known as: LCAT activator activity Relationships: is a type of enzyme activator activity [GO:0008047]; positively regulates phosphatidylcholine-sterol O-acyltransferase activity [GO:0004607]